{
  "gene_symbol": "KCNE4",
  "gene_name": "Potassium voltage-gated channel subfamily E member 4",
  "term_label": "voltage-gated potassium channel activity involved in ventricular cardiac muscle cell action potential repolarization",
  "term_id": "GO:1902282",
  "gene": "UniProtKB:Q8WWG9"
}